{
  "gene_name": "Sal-like protein 2",
  "term_id": "GO:0005634",
  "gene_symbol": "SALL2",
  "gene": "UniProtKB:Q9Y467",
  "term_label": "nucleus"
}